symbiont-mediated perturbation of host T-cell mediated immune response [GO:0052156] (biological process) Subtypes: symbiont-mediated suppression of host T-cell mediated immune response [GO:0052085] Sources: GOC:mtg_pamgo_17jul06 Definition: A process in which a symbiont alters or subverts the T-cell mediated immune response of the host organism. The host is defined as the larger of the organisms involved in a symbiotic interaction. Also known as: modulation by organism of T-cell mediated immune response of other organism involved in symbiotic interaction, modulation by symbiont of host T-cell mediated immune response, perturbation of host T-cell mediated immune response, symbiont-mediated modulation of host cell-mediated immune response, symbiont-mediated perturbation of host cell-mediated immune response Relationships: is a type of symbiont-mediated perturbation of host immune response [GO:0052553]